protein kinase complex [GO:1902911] (cellular component) Definition: A protein complex which is capable of protein kinase activity. Relationships: is a type of transferase complex, transferring phosphorus-containing groups [GO:0061695] Subtypes: GO:0005899, protein histidine kinase complex [GO:0009365], nucleotide-activated protein kinase complex [GO:0031588], Las1 complex [GO:0090730], GO:0097076, PAK family kinase-Sog2 complex [GO:0099125], Cdr2 medial cortical node complex [GO:0110115], serine/threonine protein kinase complex [GO:1902554], PKM2 protein kinase complex [GO:1990360] References: PMID:24606918 Sources: GOC:TermGenie, GOC:bhm, GO_REF:0000088 Note: An example of this is PKM2 in human (P14618) in PMID:24606918 (inferred from direct assay).